{
  "gene_name": "Uncharacterized protein C9orf152",
  "gene": "UniProtKB:Q5JTZ5",
  "gene_symbol": "C9orf152",
  "term_label": "Unknown cellular component",
  "term_id": "UNKNOWN:0003"
}